{
  "gene": "UniProtKB:P41221",
  "term_id": "GO:0005109",
  "gene_symbol": "WNT5A",
  "term_label": "frizzled binding",
  "gene_name": "Protein Wnt-5a"
}